{
  "gene_symbol": "DEDD2",
  "gene": "UniProtKB:Q8WXF8",
  "term_id": "GO:0005730",
  "term_label": "nucleolus",
  "gene_name": "DNA-binding death effector domain-containing protein 2"
}